negative regulation of ent-pimara-8(14),15-diene biosynthetic process [GO:1901543] (biological process) Also known as: down regulation of ent-pimara-8(14),15-diene anabolism, down regulation of ent-pimara-8(14),15-diene biosynthesis, down regulation of ent-pimara-8(14),15-diene biosynthetic process, down regulation of ent-pimara-8(14),15-diene formation, down regulation of ent-pimara-8(14),15-diene synthesis, down-regulation of ent-pimara-8(14),15-diene anabolism, down-regulation of ent-pimara-8(14),15-diene biosynthesis, down-regulation of ent-pimara-8(14),15-diene biosynthetic process, down-regulation of ent-pimara-8(14),15-diene formation, down-regulation of ent-pimara-8(14),15-diene synthesis, downregulation of ent-pimara-8(14),15-diene anabolism, downregulation of ent-pimara-8(14),15-diene biosynthesis, downregulation of ent-pimara-8(14),15-diene biosynthetic process, downregulation of ent-pimara-8(14),15-diene formation, downregulation of ent-pimara-8(14),15-diene synthesis, negative regulation of ent-pimara-8(14),15-diene anabolism, negative regulation of ent-pimara-8(14),15-diene biosynthesis, negative regulation of ent-pimara-8(14),15-diene formation, negative regulation of ent-pimara-8(14),15-diene synthesis, inhibition of ent-pimara-8(14),15-diene anabolism, inhibition of ent-pimara-8(14),15-diene biosynthesis, inhibition of ent-pimara-8(14),15-diene biosynthetic process, inhibition of ent-pimara-8(14),15-diene formation, inhibition of ent-pimara-8(14),15-diene synthesis Definition: Any process that stops, prevents or reduces the frequency, rate or extent of ent-pimara-8(14),15-diene biosynthetic process. Sources: GOC:TermGenie, GOC:di Relationships: is a type of negative regulation of isoprenoid metabolic process [GO:0045827]; is a type of negative regulation of lipid biosynthetic process [GO:0051055]; is a type of GO:1901542; negatively regulates ent-pimara-8(14),15-diene biosynthetic process [GO:1901541]